{
  "term_label": "late endosome",
  "term_id": "GO:0005770",
  "gene_name": "Putative DENN domain-containing protein 10 B",
  "gene": "UniProtKB:Q6NSW5",
  "gene_symbol": "DENND10P1"
}